{
  "term_label": "Unknown molecular function",
  "gene_name": "Leucine-rich repeat-containing protein 70",
  "term_id": "UNKNOWN:0001",
  "gene_symbol": "LRRC70",
  "gene": "UniProtKB:Q7Z2Q7"
}